{
  "gene_name": "Acyl-coenzyme A thioesterase 2, mitochondrial",
  "gene": "UniProtKB:P49753",
  "gene_symbol": "ACOT2",
  "term_id": "GO:0006631",
  "term_label": "fatty acid metabolic process"
}